{
  "term_id": "GO:0005811",
  "term_label": "lipid droplet",
  "gene_name": "Patatin-like phospholipase domain-containing protein 2",
  "gene_symbol": "PNPLA2",
  "gene": "UniProtKB:Q96AD5"
}